{
  "gene": "UniProtKB:P0DJR0",
  "term_id": "GO:0003924",
  "gene_symbol": "GIMD1",
  "gene_name": "GTPase IMAP family member GIMD1",
  "term_label": "GTPase activity"
}